non-canonical inflammasome complex [GO:0160074] (cellular component) References: PMID:33187725 Relationships: is a type of GO:0032991; BFO_0000050 cytosol [GO:0005829] Definition: An inflammasome complex containing CASP4, known as caspase-11 (Casp11) in mouse, which assembles upon cytosolic lipopolysaccharide-binding and directly activates Gasdermin-D (GSDMD).